{
  "gene": "UniProtKB:O75914",
  "term_label": "regulation of MAPK cascade",
  "gene_name": "Serine_threonine-protein kinase PAK 3",
  "term_id": "GO:0043408",
  "gene_symbol": "PAK3"
}